{
  "term_id": "UNKNOWN:0003",
  "gene": "UniProtKB:Q9BVK8",
  "gene_name": "BOS complex subunit TMEM147",
  "term_label": "Unknown cellular component",
  "gene_symbol": "TMEM147"
}